{
  "gene_name": "C-type lectin domain family 5 member A",
  "term_id": "GO:0045087",
  "term_label": "innate immune response",
  "gene": "UniProtKB:Q9NY25",
  "gene_symbol": "CLEC5A"
}